{
  "gene": "UniProtKB:Q86WG3",
  "gene_name": "Caytaxin",
  "gene_symbol": "ATCAY",
  "term_id": "GO:0006915",
  "term_label": "apoptotic process"
}